{
  "term_label": "I band",
  "term_id": "GO:0031674",
  "gene": "UniProtKB:P0CAP1",
  "gene_symbol": "MYZAP",
  "gene_name": "Myocardial zonula adherens protein"
}